{
  "gene_name": "Peptide deformylase, mitochondrial",
  "term_label": "peptide deformylase activity",
  "gene_symbol": "PDF",
  "term_id": "GO:0042586",
  "gene": "UniProtKB:Q9HBH1"
}